alphav-beta3 integrin-thrombospondin complex [GO:0070017] (cellular component) Relationships: is a type of plasma membrane protein complex [GO:0098797] Definition: A protein complex that consists of an alphav-beta3 integrin complex bound to thrombospondin. References: PMID:2478219 Also known as: ITGAV-ITGB3-THBS1 complex